{
  "term_id": "UNKNOWN:0002",
  "gene_symbol": "URAD",
  "gene": "UniProtKB:A6NGE7",
  "term_label": "Unknown biological process",
  "gene_name": "Putative 2-oxo-4-hydroxy-4-carboxy-5-ureidoimidazoline decarboxylase"
}